{
  "term_id": "UNKNOWN:0001",
  "gene_name": "Putative claudin-25",
  "term_label": "Unknown molecular function",
  "gene_symbol": "CLDN25",
  "gene": "UniProtKB:C9JDP6"
}